{
  "term_label": "detection of chemical stimulus involved in sensory perception of smell",
  "gene_symbol": "OR10G9",
  "gene": "UniProtKB:Q8NGN4",
  "term_id": "GO:0050911",
  "gene_name": "Olfactory receptor 10G9"
}